{
  "gene_name": "Integral membrane protein GPR137B",
  "gene_symbol": "GPR137B",
  "term_label": "lysosomal membrane",
  "gene": "UniProtKB:O60478",
  "term_id": "GO:0005765"
}